negative regulation of membrane repolarization during atrial cardiac muscle cell action potential [GO:1905001] (biological process) Also known as: down regulation of membrane repolarization during atrial cardiac muscle cell action potential, down-regulation of membrane repolarization during atrial cardiac muscle cell action potential, downregulation of membrane repolarization during atrial cardiac muscle cell action potential, inhibition of membrane repolarization during atrial cardiac muscle cell action potential, down regulation of atrial repolarization, down regulation of electrocardiogram QRS complex, down-regulation of atrial repolarization, down-regulation of electrocardiogram QRS complex, downregulation of atrial repolarization, downregulation of electrocardiogram QRS complex, inhibition of atrial repolarization, inhibition of electrocardiogram QRS complex, negative regulation of atrial repolarization, negative regulation of electrocardiogram QRS complex References: PMID:21098446 Sources: GOC:BHF, GOC:BHF_miRNA, GOC:TermGenie, GOC:mtg_cardiac_conduct_nov11, GOC:rph Relationships: is a type of GO:1905000; is a type of negative regulation of membrane repolarization during cardiac muscle cell action potential [GO:1905032]; negatively regulates membrane repolarization during atrial cardiac muscle cell action potential [GO:0098914] Definition: Any process that stops, prevents or reduces the frequency, rate or extent of membrane repolarization during atrial cardiac muscle cell action potential.